cyclohexylamine oxidase activity [GO:0018527] (molecular function) Definition: Catalysis of the reaction: cyclohexylamine + O2 + H2O = cyclohexanone + NH3 + hydrogen peroxide. References: PMID:18451 Sources: RHEA:18433 Also known as: cyclohexylamine:oxygen oxidoreductase (deaminating) Relationships: is a type of primary methylamine oxidase activity [GO:0008131]